{
  "gene_symbol": "IRAK2",
  "gene": "UniProtKB:O43187",
  "gene_name": "Interleukin-1 receptor-associated kinase-like 2",
  "term_id": "GO:0043123",
  "term_label": "positive regulation of canonical NF-kappaB signal transduction"
}